{
  "gene_symbol": "NEDD4",
  "gene_name": "E3 ubiquitin-protein ligase NEDD4",
  "gene": "UniProtKB:P46934",
  "term_id": "GO:0031623",
  "term_label": "receptor internalization"
}